{
  "gene_name": "Ephrin type-A receptor 8",
  "gene": "UniProtKB:P29322",
  "gene_symbol": "EPHA8",
  "term_id": "GO:0048013",
  "term_label": "ephrin receptor signaling pathway"
}